{
  "term_label": "Unknown cellular component",
  "gene_name": "Zinc finger protein 235",
  "gene": "UniProtKB:Q14590",
  "term_id": "UNKNOWN:0003",
  "gene_symbol": "ZNF235"
}